{
  "gene_name": "HCLS1-associated protein X-1",
  "gene": "UniProtKB:O00165",
  "term_label": "signaling adaptor activity",
  "term_id": "GO:0035591",
  "gene_symbol": "HAX1"
}